abscisic acid biosynthetic process [GO:0009688] (biological process) Relationships: is a type of abscisic acid metabolic process [GO:0009687]; is a type of sesquiterpenoid biosynthetic process [GO:0016106]; is a type of apocarotenoid biosynthetic process [GO:0043289]; is a type of monocarboxylic acid biosynthetic process [GO:0072330]; is a type of olefinic compound biosynthetic process [GO:0120255]; is a type of tertiary alcohol biosynthetic process [GO:1902645] Sources: ISBN:0387969845 Regulation: regulated by GO:0010115; positively regulated by positive regulation of abscisic acid biosynthetic process [GO:0010116]; negatively regulated by negative regulation of abscisic acid biosynthetic process [GO:0090359] Also known as: abscisic acid anabolism, abscisic acid biosynthesis, abscisic acid formation, abscisic acid synthesis Definition: The chemical reactions and pathways resulting in the formation of abscisic acid, 5-(1-hydroxy-2,6,6,trimethyl-4-oxocyclohex-2-en-1-y1)-3-methylpenta-2,4-dienoic acid.